{
  "gene_name": "Armadillo repeat-containing protein 5",
  "term_label": "anatomical structure morphogenesis",
  "term_id": "GO:0009653",
  "gene": "UniProtKB:Q96C12",
  "gene_symbol": "ARMC5"
}